{
  "term_label": "nucleus",
  "term_id": "GO:0005634",
  "gene_name": "Serine_threonine-protein phosphatase 6 regulatory subunit 3",
  "gene": "UniProtKB:Q5H9R7",
  "gene_symbol": "PPP6R3"
}